{
  "gene_symbol": "PRSS8",
  "term_id": "GO:0016485",
  "gene": "UniProtKB:Q16651",
  "gene_name": "Prostasin",
  "term_label": "protein processing"
}